{
  "term_label": "frizzled binding",
  "gene_name": "Protein Wnt-9b",
  "gene_symbol": "WNT9B",
  "gene": "UniProtKB:O14905",
  "term_id": "GO:0005109"
}